{
  "gene_symbol": "CTAGE15",
  "gene": "UniProtKB:A4D2H0",
  "term_label": "endoplasmic reticulum membrane",
  "gene_name": "cTAGE family member 15",
  "term_id": "GO:0005789"
}